{
  "term_label": "minor groove of adenine-thymine-rich DNA binding",
  "gene_name": "High mobility group protein HMG-I_HMG-Y",
  "gene": "UniProtKB:P17096",
  "gene_symbol": "HMGA1",
  "term_id": "GO:0003680"
}